{
  "gene": "UniProtKB:Q76MJ5",
  "term_label": "unfolded protein binding",
  "gene_symbol": "ERN2",
  "term_id": "GO:0051082",
  "gene_name": "Serine_threonine-protein kinase_endoribonuclease IRE2"
}